{
  "gene_name": "Putative transmenbrane protein RNF32-DT",
  "term_label": "Unknown molecular function",
  "gene": "UniProtKB:Q8NI28",
  "gene_symbol": "RNF32-DT",
  "term_id": "UNKNOWN:0001"
}